{
  "term_id": "GO:0031428",
  "gene": "UniProtKB:A6NHQ2",
  "gene_symbol": "FBLL1",
  "gene_name": "rRNA_tRNA 2'-O-methyltransferase fibrillarin-like protein 1",
  "term_label": "box C/D methylation guide snoRNP complex"
}